{
  "gene": "UniProtKB:Q8TEA1",
  "term_label": "RNA methylation",
  "term_id": "GO:0001510",
  "gene_name": "tRNA (cytosine(72)-C(5))-methyltransferase NSUN6",
  "gene_symbol": "NSUN6"
}